{
  "term_label": "membrane",
  "gene_name": "Chloride intracellular channel protein 4",
  "gene": "UniProtKB:Q9Y696",
  "term_id": "GO:0016020",
  "gene_symbol": "CLIC4"
}